{
  "gene": "UniProtKB:Q8ND25",
  "term_id": "GO:0043161",
  "term_label": "proteasome-mediated ubiquitin-dependent protein catabolic process",
  "gene_name": "E3 ubiquitin-protein ligase ZNRF1",
  "gene_symbol": "ZNRF1"
}